{
  "gene_name": "Melatonin receptor type 1B",
  "gene": "UniProtKB:P49286",
  "term_id": "GO:0005886",
  "gene_symbol": "MTNR1B",
  "term_label": "plasma membrane"
}